{
  "term_id": "GO:0005886",
  "gene_name": "Adenylate cyclase type 2",
  "gene": "UniProtKB:Q08462",
  "gene_symbol": "ADCY2",
  "term_label": "plasma membrane"
}